{
  "term_id": "GO:0014704",
  "gene_symbol": "DSP",
  "gene": "UniProtKB:P15924",
  "term_label": "intercalated disc",
  "gene_name": "Desmoplakin"
}